cilium disassembly [GO:0061523] (BP) Relationships: is a type of GO:0044782; is_a GO:1903008 Note: Note that we deem cilium and microtubule-based flagellum to be equivalent. Subtypes: GO:0060404 References: PMID:17604723, PMID:27350441 Sources: GOC:cilia, GOC:dph Definition: A cellular process that results in the breakdown of a cilium. Also known as: cilium resorption